(+)-secoisolariciresinol biosynthetic process [GO:1902135] (biological process) Also known as: (+)-secoisolariciresinol anabolism, (+)-secoisolariciresinol biosynthesis, (+)-secoisolariciresinol formation, (+)-secoisolariciresinol synthesis Definition: The chemical reactions and pathways resulting in the formation of (+)-secoisolariciresinol. Relationships: is a type of lignan biosynthetic process [GO:0009807]; is a type of diol biosynthetic process [GO:0034312]; is a type of phenol-containing compound biosynthetic process [GO:0046189] References: PMID:15949826, PMID:9872995 Sources: GOC:TermGenie